quinone metabolic process [GO:1901661] (biological process) Subtypes: ubiquinone metabolic process [GO:0006743], quinone catabolic process [GO:1901662], quinone biosynthetic process [GO:1901663] Sources: GOC:TermGenie, GOC:go_curators, GOC:pr Definition: The chemical reactions and pathways involving quinone. Also known as: quinone metabolism, quinone cofactor metabolic process, quinone cofactor metabolism Relationships: is a type of ketone metabolic process [GO:0042180]